{
  "term_id": "GO:0042043",
  "gene": "UniProtKB:Q8IYJ3",
  "gene_symbol": "SYTL1",
  "gene_name": "Synaptotagmin-like protein 1",
  "term_label": "neurexin family protein binding"
}